{
  "term_label": "Pwp2p-containing subcomplex of 90S preribosome",
  "gene": "UniProtKB:Q15269",
  "gene_name": "Periodic tryptophan protein 2 homolog",
  "gene_symbol": "PWP2",
  "term_id": "GO:0034388"
}